renal tubular secretion [GO:0097254] (biological process) Subtypes: renal sodium excretion [GO:0035812], GO:0036359, renal phosphate excretion [GO:0044722], renal urate salt excretion [GO:0097744], renal zinc excretion [GO:0180002] References: PMID:25287933 Sources: GOC:rph, Wikipedia:Renal_secretion#Secretion Relationships: is a type of GO:0003014; is a type of excretion [GO:0007588] Definition: The elimination of substances from peritubular capillaries (or surrounding hemolymph in invertebrates) into the renal tubules to be incorporated subsequently into the urine. Substances that are secreted include organic anions, ammonia, potassium and drugs.